{
  "gene": "UniProtKB:Q6Q788",
  "term_label": "cholesterol efflux",
  "gene_symbol": "APOA5",
  "gene_name": "Apolipoprotein A-V",
  "term_id": "GO:0033344"
}